{
  "gene": "UniProtKB:O60832",
  "term_id": "GO:0031429",
  "gene_symbol": "DKC1",
  "gene_name": "H_ACA ribonucleoprotein complex subunit DKC1",
  "term_label": "box H/ACA snoRNP complex"
}